{
  "term_label": "nucleus",
  "gene_name": "Sentrin-specific protease 5",
  "gene": "UniProtKB:Q96HI0",
  "term_id": "GO:0005634",
  "gene_symbol": "SENP5"
}